{
  "gene_name": "Homeobox even-skipped homolog protein 2",
  "gene_symbol": "EVX2",
  "term_id": "GO:0000978",
  "term_label": "RNA polymerase II cis-regulatory region sequence-specific DNA binding",
  "gene": "UniProtKB:Q03828"
}